{
  "gene_name": "Lens fiber major intrinsic protein",
  "gene": "UniProtKB:P30301",
  "gene_symbol": "MIP",
  "term_id": "GO:0015250",
  "term_label": "water channel activity"
}